{
  "gene_name": "MICAL-like protein 2",
  "term_id": "GO:0032456",
  "gene_symbol": "MICALL2",
  "gene": "UniProtKB:Q8IY33",
  "term_label": "endocytic recycling"
}